post-translational protein acetylation [GO:0034421] (biological process) Relationships: is a type of protein acetylation [GO:0006473]; is a type of post-translational protein modification [GO:0043687] Sources: GOC:mah Also known as: post-translational protein amino acid acetylation, posttranslational protein amino acid acetylation Definition: The addition of an acetyl group to one or more amino acids in a protein, occurring after the protein has been completely translated and released from the ribosome.